{
  "gene_name": "Adhesion G protein-coupled receptor L1",
  "gene": "UniProtKB:O94910",
  "term_id": "GO:0005886",
  "gene_symbol": "ADGRL1",
  "term_label": "plasma membrane"
}